protein malonylation [GO:0044394] (biological process) Relationships: is a type of protein acylation [GO:0043543] Sources: GOC:sp Definition: The modification of a protein amino acid by the addition of a malonyl (CO-CH2-CO) group.